{
  "gene": "UniProtKB:O60861",
  "gene_symbol": "GAS7",
  "term_id": "UNKNOWN:0001",
  "gene_name": "Growth arrest-specific protein 7",
  "term_label": "Unknown molecular function"
}